{
  "gene_symbol": "ANGPT2",
  "term_label": "extracellular space",
  "gene_name": "Angiopoietin-2",
  "term_id": "GO:0005615",
  "gene": "UniProtKB:O15123"
}